cAMP/PKA signal transduction [GO:0141156] (biological process) Definition: An intracellular signaling cassette that starts with production of cyclic AMP (cAMP) by adenylate cyclase (either transmembrane or soluble), which activates protein kinase A, and ends with activation of downstream effectors such as the transcription factor CREB that further transmit the signal within the cell. References: PMID:23209152 Also known as: PKA signaling, cAMP signaling, protein kinase A signaling, cAMP/PKA signaling cassette Relationships: is a type of intracellular signaling cassette [GO:0141124] Regulation: RO_0002211 by regulation of cAMP/PKA signal transduction [GO:0141161]; negatively regulated by negative regulation of cAMP/PKA signal transduction [GO:0141162]; positively regulated by GO:0141163